U5 snRNA 3'-end processing [GO:0034476] (BP) Relationships: is a type of GO:0034472 Sources: GOC:mah Definition: Any process involved in forming the mature 3' end of a U5 snRNA molecule. Also known as: U5 snRNA 3' end processing